{
  "gene_symbol": "APBB1",
  "gene_name": "Amyloid beta precursor protein binding family B member 1",
  "term_label": "nucleus",
  "term_id": "GO:0005634",
  "gene": "UniProtKB:O00213"
}